{
  "gene_name": "Inactive caspase-12",
  "term_id": "GO:0043525",
  "term_label": "positive regulation of neuron apoptotic process",
  "gene_symbol": "CASP12",
  "gene": "UniProtKB:Q6UXS9"
}